{
  "gene_name": "Transducin-like enhancer protein 6",
  "term_id": "GO:0003714",
  "term_label": "transcription corepressor activity",
  "gene": "UniProtKB:Q9H808",
  "gene_symbol": "TLE6"
}